negative regulation of epinephrine secretion [GO:0032811] (biological process) Relationships: is a type of regulation of epinephrine secretion [GO:0014060]; is_a negative regulation of catecholamine secretion [GO:0033604]; negatively regulates epinephrine secretion [GO:0048242] Sources: GOC:vk Definition: Any process that stops, prevents, or reduces the frequency, rate or extent of the regulated release of epinephrine. Also known as: down regulation of epinephrine secretion, down-regulation of epinephrine secretion, downregulation of epinephrine secretion, negative regulation of adrenaline secretion, inhibition of epinephrine secretion